{
  "term_label": "Unknown biological process",
  "gene": "UniProtKB:Q9ULT8",
  "gene_name": "E3 ubiquitin-protein ligase HECTD1",
  "gene_symbol": "HECTD1",
  "term_id": "UNKNOWN:0002"
}